{
  "gene_symbol": "LLGL2",
  "term_label": "regulation of establishment or maintenance of cell polarity",
  "gene": "UniProtKB:Q6P1M3",
  "term_id": "GO:0032878",
  "gene_name": "LLGL scribble cell polarity complex component 2"
}